{
  "term_id": "GO:0046654",
  "gene": "UniProtKB:Q86XF0",
  "gene_symbol": "DHFR2",
  "term_label": "tetrahydrofolate biosynthetic process",
  "gene_name": "Dihydrofolate reductase 2, mitochondrial"
}